{
  "gene_symbol": "GBP6",
  "gene": "UniProtKB:Q6ZN66",
  "term_id": "GO:0042832",
  "term_label": "defense response to protozoan",
  "gene_name": "Guanylate-binding protein 6"
}